{
  "term_label": "Unknown molecular function",
  "term_id": "UNKNOWN:0001",
  "gene_name": "NEDD8 ultimate buster 1",
  "gene": "UniProtKB:Q9Y5A7",
  "gene_symbol": "NUB1"
}